(R)-pantolactone dehydrogenase (flavin) activity [GO:0047060] (molecular function) Also known as: (R)-pantolactone:acceptor oxidoreductase (flavin-containing), (R)-pantoyllactone dehydrogenase (flavin) activity, 2-dehydropantolactone reductase (flavin) activity, 2-dehydropantoyl-lactone reductase (flavin) activity Relationships: is a type of oxidoreductase activity, acting on CH-OH group of donors [GO:0016614] Sources: EC:1.1.99.27, RHEA:21004 Definition: Catalysis of the reaction: (R)-pantolactone + A = 2-dehydropantolactone + AH(2).